{
  "gene": "UniProtKB:Q13310",
  "term_label": "Unknown biological process",
  "term_id": "UNKNOWN:0002",
  "gene_symbol": "PABPC4",
  "gene_name": "Polyadenylate-binding protein 4"
}